regulation of vasoconstriction by neuronal epinephrine [GO:0003119] (biological process) Relationships: is a type of regulation of vasoconstriction by epinephrine [GO:0003115] Sources: GOC:mtg_cardio Definition: Any process that modulates the frequency, rate or extent of reductions in the diameter of blood vessels as a result of epinephrine released by nerve endings. Also known as: regulation of vasoconstriction by neuronal adrenaline